{
  "gene_name": "Protein mono-ADP-ribosyltransferase PARP6",
  "gene_symbol": "PARP6",
  "term_label": "nuclear envelope",
  "term_id": "GO:0005635",
  "gene": "UniProtKB:Q2NL67"
}